dauer entry [GO:0043053] (BP) Definition: Entry into the facultative diapause of the dauer (enduring) larval stage of nematode development. References: PMID:10077613 Sources: GOC:cab1, GOC:kmv Also known as: nematode entry into dormancy Relationships: is a type of entry into diapause [GO:0055115]; is part of dauer larval development [GO:0040024] Regulation: regulated by regulation of dauer entry [GO:1905909]; negatively regulated by GO:1905910; positively regulated by positive regulation of dauer entry [GO:1905911]